{
  "gene": "UniProtKB:P42336",
  "gene_name": "Phosphatidylinositol 4,5-bisphosphate 3-kinase catalytic subunit alpha isoform",
  "term_label": "1-phosphatidylinositol-4,5-bisphosphate 3-kinase activity",
  "term_id": "GO:0046934",
  "gene_symbol": "PIK3CA"
}